{
  "term_label": "Unknown biological process",
  "gene_name": "Tastin",
  "gene": "UniProtKB:Q12815",
  "gene_symbol": "TROAP",
  "term_id": "UNKNOWN:0002"
}